{
  "gene_name": "Bestrophin-4",
  "gene_symbol": "BEST4",
  "term_label": "plasma membrane",
  "gene": "UniProtKB:Q8NFU0",
  "term_id": "GO:0005886"
}